ribosomal large subunit export from nucleus [GO:0000055] (biological process) Sources: GOC:mah Also known as: ribosomal large subunit export from cell nucleus, ribosomal large subunit export out of nucleus, ribosomal large subunit transport from nucleus to cytoplasm, ribosomal large subunit-nucleus export, 50S ribosomal subunit export from nucleus, 60S ribosomal subunit export from nucleus Definition: The directed movement of a ribosomal large subunit from the nucleus into the cytoplasm. Relationships: is a type of ribosomal subunit export from nucleus [GO:0000054] Regulation: regulated by GO:2000203; negatively regulated by negative regulation of ribosomal large subunit export from nucleus [GO:2000204]; positively regulated by GO:2000205